{
  "gene_name": "ABI gene family member 3",
  "term_id": "GO:0048858",
  "term_label": "cell projection morphogenesis",
  "gene_symbol": "ABI3",
  "gene": "UniProtKB:Q9P2A4"
}